{
  "gene_name": "Armadillo-like helical domain-containing protein 3",
  "term_label": "Unknown biological process",
  "term_id": "UNKNOWN:0002",
  "gene": "UniProtKB:Q5T2E6",
  "gene_symbol": "ARMH3"
}